{
  "gene_symbol": "SNX22",
  "term_id": "UNKNOWN:0002",
  "term_label": "Unknown biological process",
  "gene": "UniProtKB:Q96L94",
  "gene_name": "Sorting nexin-22"
}